{
  "gene": "UniProtKB:Q9H008",
  "gene_name": "Phospholysine phosphohistidine inorganic pyrophosphate phosphatase",
  "gene_symbol": "LHPP",
  "term_label": "inorganic diphosphate phosphatase activity",
  "term_id": "GO:0004427"
}